{
  "gene_symbol": "CDH5",
  "gene_name": "Cadherin-5",
  "gene": "UniProtKB:P33151",
  "term_label": "cell migration",
  "term_id": "GO:0016477"
}